{
  "gene": "UniProtKB:Q9H223",
  "term_label": "perinuclear region of cytoplasm",
  "term_id": "GO:0048471",
  "gene_symbol": "EHD4",
  "gene_name": "EH domain-containing protein 4"
}